{
  "gene_symbol": "KCNB1",
  "gene": "UniProtKB:Q14721",
  "term_id": "GO:0008076",
  "term_label": "voltage-gated potassium channel complex",
  "gene_name": "Potassium voltage-gated channel subfamily B member 1"
}